transcription regulatory region nucleic acid binding [GO:0001067] (molecular function) Definition: Binding to a nucleic acid region that regulates a nucleic acid-based process. Such processes include transcription, DNA replication, and DNA repair. Also known as: regulatory region nucleic acid binding Subtypes: transcription cis-regulatory region binding [GO:0000976], regulatory region RNA binding [GO:0001069] Sources: GOC:txnOH Relationships: is a type of GO:0003676